{
  "term_label": "alcohol dehydrogenase (NADP+) activity",
  "gene_name": "Aflatoxin B1 aldehyde reductase member 3",
  "term_id": "GO:0008106",
  "gene": "UniProtKB:O95154",
  "gene_symbol": "AKR7A3"
}